{
  "term_id": "GO:0010133",
  "gene_symbol": "PRODH",
  "gene": "UniProtKB:O43272",
  "term_label": "L-proline catabolic process to L-glutamate",
  "gene_name": "Proline dehydrogenase 1, mitochondrial"
}